s-triazine compound catabolic process [GO:0042204] (biological process) Definition: The chemical reactions and pathways resulting in the breakdown of any s-triazine compound. These compounds include many pesticides of widespread use in agriculture, and are characterized by a symmetrical hexameric ring consisting of alternating carbon and nitrogen atoms. Also known as: s-triazine compound breakdown, s-triazine compound catabolism, s-triazine compound degradation Relationships: is_a xenobiotic catabolic process [GO:0042178] Subtypes: atrazine catabolic process [GO:0019381], cyanuric acid catabolic process [GO:0042200], N-cyclopropylmelamine catabolic process [GO:0042202] Sources: UM-BBD_pathwayID:tria